cerebellar Golgi cell to granule cell synapse [GO:0099192] (cellular component) References: PMID:26134650 Definition: A synapse formed by a cerebellar Golgi cell synapsing on to a cerebellar granule cell. Relationships: is a type of synapse [GO:0045202]